10-formyltetrahydrofolate biosynthetic process [GO:0009257] (biological process) Definition: The chemical reactions and pathways resulting in the formation of 10-formyltetrahydrofolate, the formylated derivative of tetrahydrofolate. Sources: GOC:ai Also known as: 10-formyl-THF biosynthesis, 10-formyl-THF biosynthetic process, 10-formyltetrahydrofolate anabolism, 10-formyltetrahydrofolate biosynthesis, 10-formyltetrahydrofolate formation, 10-formyltetrahydrofolate synthesis Relationships: is a type of GO:0009256; is a type of dicarboxylic acid biosynthetic process [GO:0043650]; is_a tetrahydrofolate biosynthetic process [GO:0046654]